{
  "gene": "UniProtKB:Q6IA69",
  "gene_name": "Glutamine-dependent NAD(+) synthetase",
  "gene_symbol": "NADSYN1",
  "term_label": "NAD+ synthase (glutamine-hydrolyzing) activity",
  "term_id": "GO:0003952"
}